{
  "gene_symbol": "DCAF8",
  "term_label": "cytoplasm",
  "term_id": "GO:0005737",
  "gene": "UniProtKB:Q5TAQ9",
  "gene_name": "DDB1- and CUL4-associated factor 8"
}